{
  "term_id": "GO:0007015",
  "gene_name": "Rho-related GTP-binding protein RhoJ",
  "term_label": "actin filament organization",
  "gene": "UniProtKB:Q9H4E5",
  "gene_symbol": "RHOJ"
}